glomerular parietal epithelial cell development [GO:0072016] (biological process) Subtypes: mesonephric glomerular parietal epithelial cell development [GO:0061254], GO:0072246 Sources: GOC:mtg_kidney_jan10 Also known as: Bowman's capsule development Definition: The process whose specific outcome is the progression of a glomerular parietal epithelial cell over time, from its formation to the mature structure. Glomerular parietal epithelial cells are specialized epithelial cells that form tight junctions as a barrier to protein transport. Relationships: is a type of glomerular epithelial cell development [GO:0072310]; is part of glomerular parietal epithelial cell differentiation [GO:0072139]